c-di-GMP signaling [GO:0061939] (biological process) Also known as: 3',5'-cyclic di-GMP signaling, cyclic di-(3':5')-guanosine monophosphate signaling, cyclic di-GMP signaling, cyclic diguanylate signaling Definition: Any process that mediates the transfer of information from one cell to another using c-di-GMP as the signal. References: PMID:22864416, PMID:28057864 Regulation: RO_0002211 by regulation of c-di-GMP signaling [GO:0061940]; positively regulated by positive regulation of c-di-GMP signaling [GO:0061941]; negatively regulated by GO:0061942 Relationships: is a type of GO:0007267